{
  "gene_name": "Methyl-CpG-binding protein 2",
  "gene": "UniProtKB:P51608",
  "term_id": "GO:0000122",
  "gene_symbol": "MECP2",
  "term_label": "negative regulation of transcription by RNA polymerase II"
}